{
  "gene": "UniProtKB:P29400",
  "gene_name": "Collagen alpha-5(IV) chain",
  "term_id": "GO:0031012",
  "gene_symbol": "COL4A5",
  "term_label": "extracellular matrix"
}